{
  "gene_name": "Coiled-coil domain-containing protein 78",
  "term_id": "GO:0005737",
  "term_label": "cytoplasm",
  "gene_symbol": "CCDC78",
  "gene": "UniProtKB:A2IDD5"
}